{
  "term_id": "GO:0005634",
  "gene": "UniProtKB:Q5JVG2",
  "term_label": "nucleus",
  "gene_name": "Zinc finger protein 484",
  "gene_symbol": "ZNF484"
}